{
  "gene_name": "Secretory phospholipase A2 receptor",
  "term_label": "transmembrane signaling receptor activity",
  "term_id": "GO:0004888",
  "gene": "UniProtKB:Q13018",
  "gene_symbol": "PLA2R1"
}